{
  "term_id": "GO:0000981",
  "gene_symbol": "ZNF75CP",
  "term_label": "DNA-binding transcription factor activity, RNA polymerase II-specific",
  "gene": "UniProtKB:Q92670",
  "gene_name": "Putative zinc finger protein 75C"
}